{
  "term_label": "Unknown biological process",
  "term_id": "UNKNOWN:0002",
  "gene_name": "Olfactory receptor 52N5",
  "gene": "UniProtKB:Q8NH56",
  "gene_symbol": "OR52N5"
}